{
  "term_id": "UNKNOWN:0002",
  "gene": "UniProtKB:Q8IXW0",
  "gene_name": "Lamin tail domain-containing protein 2",
  "term_label": "Unknown biological process",
  "gene_symbol": "LMNTD2"
}